diguanylate cyclase activity [GO:0052621] (molecular function) Definition: Catalysis of the reaction: 2 GTP = cyclic di-3',5'-guanylate + 2 diphosphate + 2 H+. Also known as: GTP:GTP guanylyltransferase activity Sources: EC:2.7.7.65, RHEA:24898 Relationships: is a type of nucleotidyltransferase activity [GO:0016779]